{
  "gene_symbol": "CNOT1",
  "gene": "UniProtKB:A5YKK6",
  "term_label": "molecular adaptor activity",
  "gene_name": "CCR4-NOT transcription complex subunit 1",
  "term_id": "GO:0060090"
}